{
  "gene_name": "Neogenin",
  "gene": "UniProtKB:Q92859",
  "gene_symbol": "NEO1",
  "term_id": "GO:0098609",
  "term_label": "cell-cell adhesion"
}